{
  "gene_symbol": "PLXNB1",
  "gene_name": "Plexin-B1",
  "term_label": "negative regulation of cell adhesion",
  "gene": "UniProtKB:O43157",
  "term_id": "GO:0007162"
}